{
  "gene_symbol": "MED11",
  "term_label": "Unknown biological process",
  "term_id": "UNKNOWN:0002",
  "gene": "UniProtKB:Q9P086",
  "gene_name": "Mediator of RNA polymerase II transcription subunit 11"
}